regulation of chronic inflammatory response to non-antigenic stimulus [GO:0002880] (biological process) Subtypes: negative regulation of chronic inflammatory response to non-antigenic stimulus [GO:0002881], positive regulation of chronic inflammatory response to non-antigenic stimulus [GO:0002882] Sources: GOC:add Definition: Any process that modulates the frequency, rate, or extent of a chronic inflammatory response to a non-antigenic stimulus. Relationships: is a type of regulation of chronic inflammatory response [GO:0002676]; regulates chronic inflammatory response to non-antigenic stimulus [GO:0002545]